{
  "gene": "UniProtKB:P86791",
  "term_id": "UNKNOWN:0001",
  "gene_name": "Vacuolar fusion protein CCZ1 homolog",
  "term_label": "Unknown molecular function",
  "gene_symbol": "CCZ1"
}